{
  "gene_name": "Cytochrome c oxidase copper chaperone",
  "term_label": "mitochondrial intermembrane space",
  "gene_symbol": "COX17",
  "gene": "UniProtKB:Q14061",
  "term_id": "GO:0005758"
}